{
  "gene_name": "DnaJ homolog subfamily B member 8",
  "gene_symbol": "DNAJB8",
  "term_id": "GO:0051087",
  "term_label": "protein-folding chaperone binding",
  "gene": "UniProtKB:Q8NHS0"
}